positive regulation of apoptotic process involved in mammary gland involution [GO:0060058] (biological process) Relationships: is a type of positive regulation of apoptotic process involved in morphogenesis [GO:1902339]; positively regulates apoptotic process involved in mammary gland involution [GO:0060057] References: PMID:15282149 Sources: GOC:dph, GOC:mtg_apoptosis Also known as: positive regulation of apoptosis involved in mammary gland involution Definition: Any process that activates or increases the frequency, rate or extent of cell death by apoptotic process of mammary epithelial cells during mammary gland involution.